{
  "term_id": "GO:0005634",
  "gene": "UniProtKB:Q14919",
  "gene_symbol": "DRAP1",
  "term_label": "nucleus",
  "gene_name": "Dr1-associated corepressor"
}